{
  "gene": "UniProtKB:Q5BVD1",
  "term_id": "UNKNOWN:0001",
  "term_label": "Unknown molecular function",
  "gene_name": "TPA-induced transmembrane protein",
  "gene_symbol": "TTMP"
}